{
  "gene_name": "Bromodomain adjacent to zinc finger domain protein 1A",
  "term_label": "positive regulation of DNA replication",
  "gene": "UniProtKB:Q9NRL2",
  "term_id": "GO:0045740",
  "gene_symbol": "BAZ1A"
}